{
  "term_label": "Unknown biological process",
  "gene_symbol": "MT-ND4L",
  "gene": "UniProtKB:P03901",
  "gene_name": "NADH-ubiquinone oxidoreductase chain 4L",
  "term_id": "UNKNOWN:0002"
}